establishment of body hair planar orientation [GO:0048105] (biological process) Definition: Orientation of body hairs, projections from the surface of an organism, such that the hairs all point in a uniform direction along the surface. Sources: GOC:ascb_2009, GOC:dph, GOC:jid, GOC:tb Relationships: is a type of establishment of body hair or bristle planar orientation [GO:0048104]